GABA-ergic synapse [GO:0098982] (cellular component) Definition: A synapse that uses GABA as a neurotransmitter. These synapses are typically inhibitory. Relationships: is a type of synapse [GO:0045202] Sources: GOC:dos Subtypes: symmetric, GABA-ergic, inhibitory synapse [GO:0098983]